{
  "gene": "UniProtKB:Q8IV63",
  "gene_name": "Inactive serine_threonine-protein kinase VRK3",
  "term_label": "DNA damage response",
  "term_id": "GO:0006974",
  "gene_symbol": "VRK3"
}